cellular response to strigolactone [GO:1902348] (biological process) Relationships: is a type of cellular response to lipid [GO:0071396]; is a type of cellular response to oxygen-containing compound [GO:1901701]; is a type of response to strigolactone [GO:1902347] Also known as: cellular response to strigolactone analog GR24 References: PMID:23893171 Sources: GOC:TermGenie Definition: Any process that results in a change in state or activity of a cell (in terms of movement, secretion, enzyme production, gene expression, etc.) as a result of a strigolactone stimulus.